glomerular mesangial cell fate commitment [GO:0072152] (biological process) Sources: GOC:mtg_kidney_jan10 Definition: The process in which the developmental fate of a cell becomes restricted such that it will develop into a glomerular mesangial cell. Subtypes: GO:0061264, GO:0072256 Relationships: is a type of mesangial cell fate commitment [GO:0072151]; is part of glomerular mesangial cell differentiation [GO:0072008]